{
  "term_id": "GO:0009952",
  "gene_symbol": "TDGF1",
  "gene": "UniProtKB:P13385",
  "term_label": "anterior/posterior pattern specification",
  "gene_name": "Teratocarcinoma-derived growth factor 1"
}